{
  "gene_symbol": "CTAGE15",
  "gene": "UniProtKB:A4D2H0",
  "gene_name": "cTAGE family member 15",
  "term_id": "GO:0006888",
  "term_label": "endoplasmic reticulum to Golgi vesicle-mediated transport"
}